{
  "gene_name": "Homeobox protein Hox-C6",
  "term_label": "DNA-binding transcription factor activity, RNA polymerase II-specific",
  "term_id": "GO:0000981",
  "gene": "UniProtKB:P09630",
  "gene_symbol": "HOXC6"
}